lacrimal gland development [GO:0032808] (biological process) Sources: GOC:ln Relationships: is_a GO:0048732; is part of exocrine system development [GO:0035272] Definition: The process whose specific outcome is the progression of the lacrimal gland over time, from its formation to the mature structure. The lacrimal gland produces secretions that lubricate and protect the cornea of the eye.